{
  "term_label": "regulation of inflammatory response",
  "gene_symbol": "NLRP4",
  "gene_name": "NACHT, LRR and PYD domains-containing protein 4",
  "gene": "UniProtKB:Q96MN2",
  "term_id": "GO:0050727"
}